positive regulation of collecting lymphatic vessel constriction [GO:1903816] (biological process) Also known as: positive regulation of lymphatic vessel myogenic constriction, up regulation of collecting lymphatic vessel constriction, up regulation of lymphatic vessel myogenic constriction, up-regulation of collecting lymphatic vessel constriction, up-regulation of lymphatic vessel myogenic constriction, upregulation of collecting lymphatic vessel constriction, upregulation of lymphatic vessel myogenic constriction, activation of collecting lymphatic vessel constriction, activation of lymphatic vessel myogenic constriction Definition: Any process that activates or increases the frequency, rate or extent of collecting lymphatic vessel constriction. References: PMID:23897233 Sources: GOC:TermGenie, GO_REF:0000058 Relationships: is a type of positive regulation of multicellular organismal process [GO:0051240]; is a type of GO:1903814; positively regulates collecting lymphatic vessel constriction [GO:1990192]